3-oxoacyl-[acyl-carrier-protein] reductase (NADH) activity [GO:0047025] (molecular function) Definition: Catalysis of the reaction: NAD+ + OH-acyl-[acyl-carrier protein] = NADH + H+ + B-ketoacyl-[acyl-carrier protein]. Sources: EC:1.1.1.212, MetaCyc:1.1.1.212-RXN Also known as: 3-oxoacyl-ACP reductase (NADH) activity, 3-oxoacyl-[acyl-carrier protein] reductase (NADH) activity, (3R)-3-hydroxyacyl-acyl-carrier-protein:NAD+ oxidoreductase activity, 3-oxoacyl-acyl carrier protein (reduced nicotinamide adenine dinucleotide) reductase activity, 3-oxoacyl-acyl-carrier-protein reductase (NADH) Relationships: is a type of oxidoreductase activity, acting on the CH-OH group of donors, NAD or NADP as acceptor [GO:0016616]